{
  "gene": "UniProtKB:Q9UHB7",
  "term_id": "GO:0032783",
  "gene_symbol": "AFF4",
  "gene_name": "AF4_FMR2 family member 4",
  "term_label": "super elongation complex"
}